{
  "gene_symbol": "FAM32A",
  "term_label": "Unknown molecular function",
  "term_id": "UNKNOWN:0001",
  "gene_name": "Protein FAM32A",
  "gene": "UniProtKB:Q9Y421"
}